3-oxo-5-beta-steroid 4-dehydrogenase activity [GO:0047568] (molecular function) Definition: Catalysis of the reaction: a 3-oxo-5-beta-steroid + acceptor = a 3-oxo-D4-steroid + reduced acceptor. Relationships: is a type of steroid dehydrogenase activity, acting on the CH-CH group of donors [GO:0033765] Also known as: 3-oxo-5beta-steroid 4-dehydrogenase activity, 3-oxo-5beta-steroid:(acceptor) delta4-oxidoreductase activity, 3-oxo-5beta-steroid:acceptor delta4-oxidoreductase activity, delta4-3-ketosteroid 5-beta-reductase activity Sources: EC:1.3.99.6